{
  "gene_symbol": "CAV1",
  "term_id": "GO:0070836",
  "term_label": "caveola assembly",
  "gene": "UniProtKB:Q03135",
  "gene_name": "Caveolin-1"
}